{
  "gene": "UniProtKB:Q15418",
  "gene_name": "Ribosomal protein S6 kinase alpha-1",
  "term_label": "nucleoplasm",
  "term_id": "GO:0005654",
  "gene_symbol": "RPS6KA1"
}